{
  "term_id": "GO:0009617",
  "term_label": "response to bacterium",
  "gene": "UniProtKB:A0A0B4J279",
  "gene_symbol": "TRAV21",
  "gene_name": "T cell receptor alpha variable 21"
}